{
  "gene_name": "Apolipoprotein M",
  "gene_symbol": "APOM",
  "term_label": "high-density lipoprotein particle",
  "term_id": "GO:0034364",
  "gene": "UniProtKB:O95445"
}